ribonucleoside-diphosphate reductase activity [GO:0061731] (molecular function) Also known as: ribonucleotide reductase activity, ribonucleoside 5'-diphosphate reductase activity, ribonucleotide diphosphate reductase activity, RNR, adenosylcobalamin-dependent ribonucleotide reductase activity, aerobic non-heme iron-dependent ribonucleotide reductase activity, anaerobic iron-sulfur-dependent ribonucleotide reductase activity, class I ribonucleotide reductase activity, class II ribonucleoside-diphosphate reductase activity, class II ribonucleotide reductase activity, class III ribonucleotide reductase activity, nucleoside diphosphate reductase activity, purine/pyrimidine nucleoside diphosphate reduction Regulation: negatively regulated by ribonucleoside-diphosphate reductase inhibitor activity [GO:1990846] Relationships: is a type of GO:0016728 Definition: Catalysis of the formation of 2'-deoxyribonucleoside diphosphate from ribonucleoside diphosphate, using either thioredoxin disulfide or glutaredoxin disulfide as an acceptor. References: PMID:16756507 Sources: GOC:dph, GOC:vw Subtypes: ribonucleoside-diphosphate reductase activity, thioredoxin disulfide as acceptor [GO:0004748], ribonucleoside-diphosphate reductase activity, glutaredoxin disulfide as acceptor [GO:0036175]